Knl1/Spc105 complex [GO:0180019] (cellular component) Relationships: is a type of GO:0032991; is part of outer kinetochore [GO:0000940] Definition: A kinetochore subcomplex that binds to centromeric chromatin and forms part of the outer kinetochore. It helps to recruit outer kinetochore subunits that will bind to microtubules. In humans and yeast respectively, it consists of KNL1/Spc105p and ZWINT/Kre28p. References: PMID:27881301